selenocystathionine beta-synthase activity [GO:0098605] (molecular function) References: PMID:6456763 Relationships: is a type of GO:0016836 Definition: Catalysis of the reaction: L-Serine + Selenohomocysteine = L-Selenocystathionine + H2O.